mechanosensory behavior [GO:0007638] (biological process) Relationships: is a type of behavior [GO:0007610]; is part of response to mechanical stimulus [GO:0009612] Definition: Behavior that is dependent upon the sensation of a mechanical stimulus. Also known as: behavioral response to mechanical stimulus, behavioural response to mechanical stimulus, mechanosensory behaviour Regulation: regulated by GO:1905790; negatively regulated by GO:1905791; positively regulated by positive regulation of mechanosensory behavior [GO:1905792] Subtypes: GO:0031223 Sources: GOC:go_curators